absorption of visible light [GO:0016038] (biological process) Definition: The reception of a (visible light) photon by a cell, visible light being defined as having a wavelength within the range 380-780 nm. Sources: GOC:go_curators, ISBN:0198506732 Relationships: is a type of light absorption [GO:0016037]